{
  "gene_symbol": "ACE2",
  "gene_name": "Angiotensin-converting enzyme 2",
  "term_id": "GO:0005886",
  "gene": "UniProtKB:Q9BYF1",
  "term_label": "plasma membrane"
}